{
  "term_id": "UNKNOWN:0002",
  "gene": "UniProtKB:Q8WTZ4",
  "gene_symbol": "CA5BP1",
  "term_label": "Unknown biological process",
  "gene_name": "Putative inactive carbonic anhydrase 5B-like protein"
}